{
  "gene_name": "Protein disulfide-isomerase A4",
  "gene": "UniProtKB:P13667",
  "term_id": "GO:0006457",
  "term_label": "protein folding",
  "gene_symbol": "PDIA4"
}